{
  "term_label": "potassium ion transmembrane transport",
  "gene_name": "Potassium voltage-gated channel subfamily A member 7",
  "term_id": "GO:0071805",
  "gene_symbol": "KCNA7",
  "gene": "UniProtKB:Q96RP8"
}